{
  "term_label": "DNA-binding transcription factor activity, RNA polymerase II-specific",
  "gene_name": "Double homeobox protein 4C",
  "term_id": "GO:0000981",
  "gene": "UniProtKB:Q6RFH8",
  "gene_symbol": "DUX4L9"
}